{
  "gene_symbol": "LCE1E",
  "gene": "UniProtKB:Q5T753",
  "term_label": "Unknown cellular component",
  "gene_name": "Late cornified envelope protein 1E",
  "term_id": "UNKNOWN:0003"
}